{
  "gene_symbol": "ZNF876P",
  "gene_name": "Putative zinc finger protein 876",
  "term_id": "GO:0006355",
  "gene": "UniProtKB:Q49A33",
  "term_label": "regulation of DNA-templated transcription"
}